negative regulation of somatic stem cell population maintenance [GO:1904673] (biological process) Relationships: is a type of negative regulation of stem cell population maintenance [GO:1902455]; is a type of regulation of somatic stem cell population maintenance [GO:1904672]; negatively regulates GO:0035019 Also known as: down regulation of somatic stem cell population maintenance, down-regulation of somatic stem cell population maintenance, downregulation of somatic stem cell population maintenance, inhibition of somatic stem cell population maintenance References: PMID:19409607 Sources: GOC:BHF, GOC:BHF_miRNA, GOC:TermGenie, GOC:rph, GO_REF:0000058 Definition: Any process that stops, prevents or reduces the frequency, rate or extent of somatic stem cell population maintenance. Subtypes: negative regulation of mesenchymal cell apoptotic process involved in nephron morphogenesis [GO:0072040]